{
  "gene": "UniProtKB:Q03014",
  "term_label": "regulation of transcription by RNA polymerase II",
  "gene_name": "Hematopoietically-expressed homeobox protein HHEX",
  "gene_symbol": "HHEX",
  "term_id": "GO:0006357"
}